{
  "gene": "UniProtKB:Q13310",
  "term_id": "GO:1990904",
  "term_label": "ribonucleoprotein complex",
  "gene_symbol": "PABPC4",
  "gene_name": "Polyadenylate-binding protein 4"
}